regulation of sevenless signaling pathway [GO:0045501] (biological process) Definition: Any process that modulates the frequency, rate or extent of the sevenless signaling pathway. Sources: GOC:go_curators Also known as: regulation of sev signaling pathway, regulation of sevenless signalling pathway Relationships: is a type of regulation of signal transduction [GO:0009966]; is a type of regulation of R7 cell differentiation [GO:0045676]; RO_0002211 GO:0045500 Subtypes: GO:0045873, positive regulation of sevenless signaling pathway [GO:0045874]